{
  "gene": "UniProtKB:Q96HN2",
  "term_label": "S-adenosylmethionine cycle",
  "gene_name": "Adenosylhomocysteinase 3",
  "gene_symbol": "AHCYL2",
  "term_id": "GO:0033353"
}